{
  "term_label": "microtubule motor activity",
  "gene_name": "Kinesin-like protein KIF19",
  "gene_symbol": "KIF19",
  "gene": "UniProtKB:Q2TAC6",
  "term_id": "GO:0003777"
}